mitotic interphase [GO:0051329] (BP) Also known as: interphase of mitotic cell cycle Definition: The cell cycle phase following cytokinesis which begins with G1 phase, proceeds through S phase and G2 phase and ends when mitotic prophase begins. During interphase the cell readies itself for mitosis and the replication of its DNA occurs. Sources: GOC:mtg_cell_cycle Note: Note that this term should not be used for direct annotation. If you are trying to make an annotation to x phase, it is likely that the correct annotation is 'regulation of x/y phase transition' or to a process which occurs during the reported phase (i.e mitotic DNA replication for mitotic S-phase). To capture the phase when a specific location or process is observed, the phase term can be used in an annotation extension (PMID:24885854) applied to a cellular component term (with the relation exists_during) or a biological process term (with the relation happens_during). Relationships: is a type of interphase [GO:0051325]; is a type of mitotic cell cycle phase [GO:0098763]